protein-DNA ISRE complex assembly [GO:0035362] (biological process) Definition: The aggregation, arrangement and bonding together of proteins and DNA molecules to form a protein-DNA complex, in which the complex is formed through interaction of the protein(s) with a interferon-stimulated response element (ISRE) in the DNA. Relationships: is a type of protein-DNA complex assembly [GO:0065004] References: PMID:11747630 Sources: GOC:amm Also known as: protein-DNA interferon-stimulated response element complex assembly